marneral synthase activity [GO:0034074] (molecular function) References: PMID:16425307, PMID:18033581 Sources: GOC:cb Definition: Catalysis of the reaction: oxidosqualene = marneral. Relationships: is a type of oxidosqualene cyclase activity [GO:0031559]